plasma lipoprotein particle [GO:0034358] (cellular component) Definition: A spherical particle with a hydrophobic core of triglycerides and/or cholesterol esters, surrounded by an amphipathic monolayer of phospholipids, cholesterol and apolipoproteins. Plasma lipoprotein particles transport lipids, which are non-covalently associated with the particles, in the blood or lymph. Relationships: is a type of GO:1990777; is part of GO:0005615 Subtypes: low-density lipoprotein particle [GO:0034362], GO:0034364, triglyceride-rich plasma lipoprotein particle [GO:0034385], GO:0042627 Sources: GOC:BHF, GOC:expert_pt, GOC:rl